regulation of intracellular estrogen receptor signaling pathway [GO:0033146] (biological process) Sources: GOC:mah Subtypes: negative regulation of intracellular estrogen receptor signaling pathway [GO:0033147], positive regulation of intracellular estrogen receptor signaling pathway [GO:0033148] Relationships: is a type of regulation of intracellular steroid hormone receptor signaling pathway [GO:0033143]; regulates estrogen receptor signaling pathway [GO:0030520] Also known as: regulation of estrogen receptor signaling pathway, regulation of estrogen receptor signalling pathway Definition: Any process that modulates the frequency, rate or extent of the activity of an intracellular estrogen receptor signaling pathway.